{
  "term_label": "Unknown cellular component",
  "term_id": "UNKNOWN:0003",
  "gene_symbol": "LNX2",
  "gene_name": "Ligand of Numb protein X 2",
  "gene": "UniProtKB:Q8N448"
}